{
  "gene": "UniProtKB:Q96EY7",
  "term_id": "GO:0032543",
  "gene_name": "Small ribosomal subunit protein mS39",
  "term_label": "mitochondrial translation",
  "gene_symbol": "PTCD3"
}